{
  "term_label": "positive regulation of canonical NF-kappaB signal transduction",
  "gene_name": "Interleukin-1 receptor-associated kinase 3",
  "gene_symbol": "IRAK3",
  "gene": "UniProtKB:Q9Y616",
  "term_id": "GO:0043123"
}